{
  "gene": "UniProtKB:P62699",
  "gene_name": "Protein yippee-like 5",
  "gene_symbol": "YPEL5",
  "term_id": "UNKNOWN:0001",
  "term_label": "Unknown molecular function"
}